{
  "gene_name": "Myotubularin-related protein 1",
  "gene_symbol": "MTMR1",
  "term_label": "phosphatidylinositol-3-phosphate phosphatase activity",
  "term_id": "GO:0004438",
  "gene": "UniProtKB:Q13613"
}